{
  "term_label": "ubiquitin conjugating enzyme binding",
  "term_id": "GO:0031624",
  "gene_symbol": "DCUN1D5",
  "gene_name": "DCN1-like protein 5",
  "gene": "UniProtKB:Q9BTE7"
}